{
  "term_label": "gamma-tubulin binding",
  "gene_name": "Gamma-tubulin complex component 3",
  "gene_symbol": "TUBGCP3",
  "term_id": "GO:0043015",
  "gene": "UniProtKB:Q96CW5"
}